{
  "gene_name": "Mannose-6-phosphate isomerase",
  "term_label": "cytosol",
  "gene_symbol": "MPI",
  "term_id": "GO:0005829",
  "gene": "UniProtKB:P34949"
}